{
  "gene_name": "Nuclear receptor-interacting protein 1",
  "term_id": "GO:0005634",
  "term_label": "nucleus",
  "gene": "UniProtKB:P48552",
  "gene_symbol": "NRIP1"
}